{
  "gene": "UniProtKB:Q8NGM1",
  "gene_symbol": "OR4C15",
  "term_label": "Unknown biological process",
  "gene_name": "Olfactory receptor 4C15",
  "term_id": "UNKNOWN:0002"
}